{
  "gene": "UniProtKB:Q9UNX4",
  "term_label": "small-subunit processome",
  "term_id": "GO:0032040",
  "gene_symbol": "WDR3",
  "gene_name": "WD repeat-containing protein 3"
}